{
  "gene_symbol": "RELB",
  "term_label": "nucleus",
  "gene": "UniProtKB:Q01201",
  "gene_name": "Transcription factor RelB",
  "term_id": "GO:0005634"
}